{
  "gene_symbol": "PPARG",
  "term_label": "negative regulation of inflammatory response",
  "gene_name": "Peroxisome proliferator-activated receptor gamma",
  "gene": "UniProtKB:P37231",
  "term_id": "GO:0050728"
}